{
  "term_label": "cytosolic large ribosomal subunit",
  "term_id": "GO:0022625",
  "gene_symbol": "RPL14",
  "gene_name": "Large ribosomal subunit protein eL14",
  "gene": "UniProtKB:P50914"
}